neural tissue regeneration [GO:0097719] (biological process) Definition: The regrowth of neural tissue following its loss or destruction. Also known as: neuroregeneration Relationships: is a type of tissue regeneration [GO:0042246] Sources: Wikipedia:Neuroregeneration